{
  "gene_name": "Doublesex- and mab-3-related transcription factor 2",
  "gene": "UniProtKB:Q9Y5R5",
  "term_id": "GO:0000978",
  "gene_symbol": "DMRT2",
  "term_label": "RNA polymerase II cis-regulatory region sequence-specific DNA binding"
}